{
  "gene_symbol": "NPBWR1",
  "term_label": "neuropeptide binding",
  "gene_name": "Neuropeptides B_W receptor type 1",
  "term_id": "GO:0042923",
  "gene": "UniProtKB:P48145"
}